positive regulation of toll-like receptor 9 signaling pathway by B cell receptor internalization [GO:1901245] (biological process) Definition: The movement of a B cell receptor (BCR) from the plasma membrane to the inside of the cell, which results in positive regulation of toll-like receptor 9 (TLR9) signaling. For example, internalized BCR signals to recruit TLR9 from multiple small endosomes to large autophagosome-like compartments to enhance TLR9 signaling. Relationships: is a type of positive regulation of toll-like receptor 9 signaling pathway [GO:0034165]; is a type of B cell receptor internalization [GO:0036300]; is a type of positive regulation of signal transduction by receptor internalization [GO:0038010] Also known as: positive regulation of TLR9 signaling pathway by B cell receptor internalization, positive regulation of TLR9 signaling pathway by BCR endocytosis, positive regulation of TLR9 signaling pathway by BCR receptor internalization, positive regulation of toll-like receptor 9 signaling pathway by BCR endocytosis, positive regulation of toll-like receptor 9 signaling pathway by BCR receptor internalization, positive regulation of toll-like receptor 9 signalling pathway by B cell receptor internalization, positive regulation of toll-like receptor 9 signalling pathway by BCR endocytosis, positive regulation of toll-like receptor 9 signalling pathway by BCR receptor internalization, BCR-induced TLR9 recruitment References: PMID:18513998 Sources: GOC:TermGenie, GOC:amm, GOC:bf